regulation of shoot system development [GO:0048831] (biological process) Definition: Any process that modulates the frequency, rate or extent of shoot development. References: PMID:16361392 Sources: GOC:tb Also known as: regulation of shoot development Relationships: is a type of regulation of developmental process [GO:0050793]; regulates GO:0048367 Subtypes: regulation of flower development [GO:0009909]